{
  "term_label": "nucleus",
  "term_id": "GO:0005634",
  "gene": "UniProtKB:P09525",
  "gene_symbol": "ANXA4",
  "gene_name": "Annexin A4"
}